{
  "gene_name": "PC-esterase domain-containing protein 1A",
  "term_label": "Unknown molecular function",
  "term_id": "UNKNOWN:0001",
  "gene_symbol": "PCED1A",
  "gene": "UniProtKB:Q9H1Q7"
}